{
  "term_label": "Unknown biological process",
  "gene": "UniProtKB:B6SEH8",
  "term_id": "UNKNOWN:0002",
  "gene_symbol": "ERVV-1",
  "gene_name": "Endogenous retrovirus group V member 1 Env polyprotein"
}